D-alanine-2-oxoglutarate aminotransferase activity [GO:0047810] (molecular function) Relationships: is_a transaminase activity [GO:0008483] Definition: Catalysis of the reaction: D-alanine + 2-oxoglutarate = pyruvate + D-glutamate. Also known as: D-alanine transaminase activity, D-amino acid aminotransferase activity, D-amino acid transaminase activity, D-amino-acid transaminase activity, D-alanine aminotransferase activity, D-alanine-D-glutamate transaminase activity, D-aspartate aminotransferase activity, D-aspartate transaminase activity, D-aspartic aminotransferase activity Sources: EC:2.6.1.21